{
  "gene_name": "Neuronal regeneration-related protein",
  "gene_symbol": "NREP",
  "term_label": "Unknown cellular component",
  "term_id": "UNKNOWN:0003",
  "gene": "UniProtKB:Q16612"
}